mesenchymal stem cell differentiation [GO:0072497] (biological process) Sources: CL:0002452, GOC:BHF Definition: The process in which a relatively unspecialized cell acquires specialized features of a mesenchymal stem cell. A mesenchymal stem cell is a cell that retains the ability to divide and proliferate throughout life to provide progenitor cells that can differentiate into specialized mesenchymal cells. Relationships: is a type of stem cell differentiation [GO:0048863] Regulation: RO_0002211 by GO:2000739; negatively regulated by negative regulation of mesenchymal stem cell differentiation [GO:2000740]; positively regulated by GO:2000741 Subtypes: mesenchymal stem cell differentiation involved in nephron morphogenesis [GO:0072037], amniotic stem cell differentiation [GO:0097086]